{
  "term_label": "immunoglobulin mediated immune response",
  "gene": "UniProtKB:A0A0B4J1V6",
  "term_id": "GO:0016064",
  "gene_symbol": "IGHV3-73",
  "gene_name": "Immunoglobulin heavy variable 3-73"
}